{
  "gene": "UniProtKB:Q6NSI8",
  "term_id": "GO:0045190",
  "gene_symbol": "SANBR",
  "gene_name": "SANT and BTB domain regulator of class switch recombination",
  "term_label": "isotype switching"
}